{
  "gene_name": "Aminoacyl tRNA synthase complex-interacting multifunctional protein 2",
  "gene_symbol": "AIMP2",
  "term_id": "UNKNOWN:0002",
  "gene": "UniProtKB:Q13155",
  "term_label": "Unknown biological process"
}